{
  "term_label": "cytoplasm",
  "term_id": "GO:0005737",
  "gene_name": "Adipogenin",
  "gene_symbol": "ADIG",
  "gene": "UniProtKB:Q0VDE8"
}